positive regulation of testosterone secretion [GO:2000845] (biological process) Definition: Any process that activates or increases the frequency, rate or extent of testosterone secretion. Relationships: is a type of GO:0032370; is a type of GO:0046887; is a type of regulation of testosterone secretion [GO:2000843]; positively regulates testosterone secretion [GO:0035936] Sources: GOC:sl